{
  "gene_symbol": "MRPL35",
  "term_label": "Unknown molecular function",
  "term_id": "UNKNOWN:0001",
  "gene": "UniProtKB:Q9NZE8",
  "gene_name": "Large ribosomal subunit protein bL35m"
}